{
  "gene": "UniProtKB:Q9Y2G2",
  "term_label": "nucleus",
  "gene_name": "Caspase recruitment domain-containing protein 8",
  "gene_symbol": "CARD8",
  "term_id": "GO:0005634"
}